{
  "term_id": "GO:0003690",
  "gene_symbol": "IFI16",
  "gene": "UniProtKB:Q16666",
  "term_label": "double-stranded DNA binding",
  "gene_name": "Gamma-interferon-inducible protein 16"
}